{
  "gene_symbol": "WHRN",
  "term_id": "GO:0007605",
  "gene": "UniProtKB:Q9P202",
  "term_label": "sensory perception of sound",
  "gene_name": "Whirlin"
}